{
  "gene_name": "Collagen and calcium-binding EGF domain-containing protein 1",
  "gene_symbol": "CCBE1",
  "gene": "UniProtKB:Q6UXH8",
  "term_label": "extracellular space",
  "term_id": "GO:0005615"
}